{
  "gene": "UniProtKB:Q9HB71",
  "gene_name": "Calcyclin-binding protein",
  "term_id": "GO:0060090",
  "term_label": "molecular adaptor activity",
  "gene_symbol": "CACYBP"
}